{
  "gene_name": "Schwannomin-interacting protein 1",
  "gene_symbol": "SCHIP1",
  "term_label": "cell junction",
  "term_id": "GO:0030054",
  "gene": "UniProtKB:P0DPB3"
}